{
  "gene_name": "TYRO protein tyrosine kinase-binding protein",
  "gene": "UniProtKB:O43914",
  "term_label": "signaling receptor binding",
  "gene_symbol": "TYROBP",
  "term_id": "GO:0005102"
}